positive regulation of somatic stem cell division [GO:1904677] (biological process) Relationships: is a type of positive regulation of cell division [GO:0051781]; is a type of regulation of somatic stem cell division [GO:1904675]; positively regulates somatic stem cell division [GO:0048103] Definition: Any process that activates or increases the frequency, rate or extent of somatic stem cell division. Also known as: positive regulation of somatic stem cell renewal, up regulation of somatic stem cell division, up regulation of somatic stem cell renewal, up-regulation of somatic stem cell division, up-regulation of somatic stem cell renewal, upregulation of somatic stem cell division, upregulation of somatic stem cell renewal, activation of somatic stem cell division, activation of somatic stem cell renewal References: PMID:19409607 Sources: GOC:BHF, GOC:BHF_miRNA, GOC:TermGenie, GOC:rph, GO_REF:0000058